{
  "gene_name": "1-acylglycerol-3-phosphate O-acyltransferase PNPLA3",
  "term_id": "GO:0016020",
  "gene_symbol": "PNPLA3",
  "term_label": "membrane",
  "gene": "UniProtKB:Q9NST1"
}